regulation of beta-glucan biosynthetic process [GO:0032951] (biological process) Sources: GOC:mah Relationships: is a type of regulation of glucan biosynthetic process [GO:0010962]; is a type of regulation of beta-glucan metabolic process [GO:0032950]; regulates beta-glucan biosynthetic process [GO:0051274] Definition: Any process that modulates the frequency, rate or extent of the chemical reactions and pathways relusting in the formation of beta-glucans. Also known as: regulation of beta-glucan anabolism, regulation of beta-glucan biosynthesis, regulation of beta-glucan formation, regulation of beta-glucan synthesis Subtypes: regulation of (1->3)-beta-D-glucan biosynthetic process [GO:0032953], GO:0060917, GO:0090093, regulation of cellulose biosynthetic process [GO:2001006]